actin crosslink formation [GO:0051764] (biological process) Also known as: actin crosslinking, formation of actin crosslink, bridging actin filaments, actin bundling Relationships: is a type of actin filament organization [GO:0007015] Note: See also the molecular function term 'protein binding, bridging ; GO:0030674'. Sources: GOC:ai Definition: The process in which two or more actin filaments are connected together by proteins that act as crosslinks between the filaments. The crosslinked filaments may be on the same or differing axes.